{
  "term_id": "GO:0030258",
  "gene_name": "Lysophospholipid acyltransferase 1",
  "term_label": "lipid modification",
  "gene": "UniProtKB:Q6ZNC8",
  "gene_symbol": "MBOAT1"
}